{
  "gene_name": "ORC ubiquitin ligase 1",
  "term_label": "regulation of DNA replication",
  "gene": "UniProtKB:Q5W0B1",
  "term_id": "GO:0006275",
  "gene_symbol": "OBI1"
}